capsomere [GO:0046727] (cellular component) Also known as: capsomer Subtypes: viral capsid, major subunit [GO:0098017], viral capsid, minor subunit [GO:0098018] Sources: ISBN:0198506732 Definition: Any of the protein subunits that comprise the closed shell or coat (capsid) of certain viruses. Relationships: is a type of GO:0044423; is part of GO:0019028